ubiquitin-protein transferase inhibitor activity [GO:0055105] (molecular function) Definition: Binds to and stops, prevents or reduces the activity of a ubiquitin-protein transferase. Relationships: is a type of enzyme inhibitor activity [GO:0004857]; is a type of ubiquitin-protein transferase regulator activity [GO:0055106]; negatively regulates GO:0004842 Subtypes: ubiquitin ligase inhibitor activity [GO:1990948] Sources: GOC:BHF, GOC:rl